{
  "term_id": "GO:0000981",
  "gene_symbol": "ZIK1",
  "gene_name": "Zinc finger protein interacting with ribonucleoprotein K",
  "gene": "UniProtKB:Q3SY52",
  "term_label": "DNA-binding transcription factor activity, RNA polymerase II-specific"
}